{
  "term_id": "GO:0000981",
  "gene_symbol": "ZNF280C",
  "term_label": "DNA-binding transcription factor activity, RNA polymerase II-specific",
  "gene": "UniProtKB:Q8ND82",
  "gene_name": "Zinc finger protein 280C"
}